positive regulation of pattern recognition receptor signaling pathway [GO:0062208] (biological process) Definition: Any process that decreases the rate, frequency or extent of a pattern recognition receptor signaling pathway. Relationships: is a type of positive regulation of signal transduction [GO:0009967]; is a type of positive regulation of innate immune response [GO:0045089]; is a type of regulation of pattern recognition receptor signaling pathway [GO:0062207]; positively regulates pattern recognition receptor signaling pathway [GO:0002221] References: PMID:30610168 Subtypes: positive regulation of toll-like receptor signaling pathway [GO:0034123], positive regulation of toll-like receptor 1 signaling pathway [GO:0034133], GO:0034137, positive regulation of toll-like receptor 3 signaling pathway [GO:0034141], GO:0034145, positive regulation of toll-like receptor 5 signaling pathway [GO:0034149], positive regulation of toll-like receptor 6 signaling pathway [GO:0034153], GO:0034157, positive regulation of toll-like receptor 8 signaling pathway [GO:0034161], positive regulation of toll-like receptor 9 signaling pathway [GO:0034165], positive regulation of toll-like receptor 10 signaling pathway [GO:0034169], positive regulation of toll-like receptor 11 signaling pathway [GO:0034173], GO:0034177, positive regulation of toll-like receptor 13 signaling pathway [GO:0034181], positive regulation of peptidoglycan recognition protein signaling pathway [GO:0061059], positive regulation of nucleotide-binding domain, leucine rich repeat containing receptor signaling pathway [GO:0070426], positive regulation of inflammasome-mediated signaling pathway [GO:0141087], GO:0141111, GO:1900245, GO:1900246, positive regulation of toll-like receptor 15 signaling pathway [GO:2000442]